{
  "gene_name": "Putative inactive carbonic anhydrase 5B-like protein",
  "gene_symbol": "CA5BP1",
  "gene": "UniProtKB:Q8WTZ4",
  "term_label": "carbonate dehydratase activity",
  "term_id": "GO:0004089"
}